NAGS/NAGK complex [GO:0106098] (cellular component) References: PMID:11553611 Sources: GOC:lnp Relationships: is a type of protein acetyltransferase complex [GO:0031248]; is_a GO:0061695; is_a mitochondrial protein-containing complex [GO:0098798]; is part of mitochondrial matrix [GO:0005759] Definition: A protein complex that acts both as N-acetylglutamate synthase (NAGS) catalysing the production of N-Acetylglutamate from glutamate and acetyl-CoA, and as N-acetylglutamate kinase (NAGK) catalysing the reaction ATP + N-acetyl-L-glutamate = ADP + N-acetyl-L-glutamyl 5-phosphate.